MHC class Ib protein binding, via antigen binding groove [GO:0023030] (MF) Relationships: is a type of GO:0023029; BFO_0000050 GO:0023025 Definition: Binding to a major histocompatibility complex class Ib molecules via the antigen binding groove. Sources: GOC:mtg_signal, GOC:vw